{
  "term_label": "Unknown biological process",
  "term_id": "UNKNOWN:0002",
  "gene_symbol": "GDAP1L1",
  "gene": "UniProtKB:Q96MZ0",
  "gene_name": "Ganglioside-induced differentiation-associated protein 1-like 1"
}